{
  "gene_symbol": "SPIRE2",
  "gene": "UniProtKB:Q8WWL2",
  "gene_name": "Protein spire homolog 2",
  "term_id": "GO:0008017",
  "term_label": "microtubule binding"
}